{
  "gene_name": "Hsp90 co-chaperone Cdc37",
  "term_label": "cytoplasm",
  "gene": "UniProtKB:Q16543",
  "gene_symbol": "CDC37",
  "term_id": "GO:0005737"
}